{
  "term_id": "GO:0030198",
  "gene_name": "A disintegrin and metalloproteinase with thrombospondin motifs 2",
  "term_label": "extracellular matrix organization",
  "gene_symbol": "ADAMTS2",
  "gene": "UniProtKB:O95450"
}